spermidine deacetylation [GO:0106048] (biological process) Also known as: N8-acetylspermidine deacetylation References: PMID:28516954 Definition: The modification of acetylspermadine by the removal of acetyl groups. Relationships: is a type of GO:0008216; is a type of polyamine deacetylation [GO:0106047]